{
  "gene": "UniProtKB:Q02750",
  "gene_name": "Dual specificity mitogen-activated protein kinase kinase 1",
  "term_id": "UNKNOWN:0003",
  "term_label": "Unknown cellular component",
  "gene_symbol": "MAP2K1"
}